{
  "gene_symbol": "PXN",
  "gene_name": "Paxillin",
  "term_id": "GO:0005911",
  "term_label": "cell-cell junction",
  "gene": "UniProtKB:P49023"
}